{
  "gene_name": "ATP-dependent DNA_RNA helicase DHX36",
  "gene": "UniProtKB:Q9H2U1",
  "term_id": "GO:0005634",
  "term_label": "nucleus",
  "gene_symbol": "DHX36"
}